{
  "term_id": "UNKNOWN:0001",
  "gene": "UniProtKB:P0CL81",
  "term_label": "Unknown molecular function",
  "gene_symbol": "GAGE12G",
  "gene_name": "G antigen 12G"
}